lactosylceramide beta-1,3-galactosyltransferase activity [GO:0047240] (molecular function) Sources: EC:2.4.1.179, RHEA:18413 Definition: Catalysis of the reaction: D-galactosyl-(1->4)-beta-D-glucosyl-R + UDP-D-galactose = D-galactosyl-(1->3)-beta-D-galactosyl-(1->4)-beta-D-glucosyl-R + H+ + UDP. Relationships: is a type of UDP-galactosyltransferase activity [GO:0035250]; is_a beta-1,3-galactosyltransferase activity [GO:0048531] Also known as: UDP-galactose:D-galactosyl-1,4-beta-D-glucosyl-R beta-1,3-galactosyltransferase activity, UDPgalactose:D-galactosyl-1,4-beta-D-glucosyl-R beta-1,3-galactosyltransferase activity, uridine diphosphogalactose-lactosylceramide beta1->3-galactosyltransferase activity